{
  "gene_name": "Inactive serine_threonine-protein kinase PLK5",
  "gene_symbol": "PLK5",
  "term_id": "GO:0006974",
  "gene": "UniProtKB:Q496M5",
  "term_label": "DNA damage response"
}